detection of activity [GO:0014865] (biological process) Definition: The series of events in which an activity stimulus is received by a cell and converted into a molecular signal. Sources: GOC:mtg_muscle Subtypes: detection of muscle activity [GO:0014864] Relationships: is a type of response to activity [GO:0014823]; is a type of detection of stimulus [GO:0051606]